{
  "gene": "UniProtKB:P0CW18",
  "gene_symbol": "PRSS56",
  "term_id": "GO:0004252",
  "term_label": "serine-type endopeptidase activity",
  "gene_name": "Serine protease 56"
}